positive regulation of endothelial cell chemotaxis by VEGF-activated vascular endothelial growth factor receptor signaling pathway [GO:0038033] (biological process) Relationships: is a type of GO:0038089; is a type of GO:0048010; is a type of positive regulation of endothelial cell chemotaxis [GO:2001028] Definition: The series of molecular signals initiated by the binding of a vascular endothelial growth factor (VEGF) to its receptor on the surface of a cell, which activates or increases the frequency, rate or extent of endothelial cell chemotaxis. Also known as: VEGF-mediated chemotactic endothelial cell migration, VEGF-VEGFR-induced endothelial cell chemotaxis, positive regulation of endothelial cell chemotaxis by VEGF-activated vascular endothelial growth factor receptor signalling pathway, positive regulation of endothelial cell chemotaxis by VEGF/VEGFR signaling pathway, vascular endothelial growth factor receptor signaling pathway involved in endothelial cell chemotaxis References: PMID:21245381 Sources: GOC:BHF, GOC:bf, GOC:rl